{
  "term_id": "UNKNOWN:0002",
  "term_label": "Unknown biological process",
  "gene_symbol": "SCGB1D4",
  "gene_name": "Secretoglobin family 1D member 4",
  "gene": "UniProtKB:Q6XE38"
}